{
  "term_id": "UNKNOWN:0003",
  "gene_symbol": "ERVMER34-1",
  "gene": "UniProtKB:Q9H9K5",
  "term_label": "Unknown cellular component",
  "gene_name": "Endogenous retroviral envelope protein HEMO"
}